{
  "term_id": "UNKNOWN:0003",
  "gene_name": "Protein ARK2N",
  "term_label": "Unknown cellular component",
  "gene_symbol": "ARK2N",
  "gene": "UniProtKB:Q96B23"
}